{
  "term_id": "UNKNOWN:0001",
  "gene_name": "Putative protein RIG",
  "gene_symbol": "RIG",
  "term_label": "Unknown molecular function",
  "gene": "UniProtKB:Q13278"
}